{
  "term_id": "GO:1902093",
  "term_label": "positive regulation of flagellated sperm motility",
  "gene_name": "Neuromedin-K receptor",
  "gene": "UniProtKB:P29371",
  "gene_symbol": "TACR3"
}